{
  "gene_name": "Protein HID1",
  "gene": "UniProtKB:Q8IV36",
  "term_id": "GO:0000138",
  "gene_symbol": "HID1",
  "term_label": "Golgi trans cisterna"
}